{
  "gene_symbol": "TNFRSF13C",
  "gene_name": "Tumor necrosis factor receptor superfamily member 13C",
  "term_id": "UNKNOWN:0001",
  "term_label": "Unknown molecular function",
  "gene": "UniProtKB:Q96RJ3"
}